{
  "gene_symbol": "KLHL38",
  "gene_name": "Kelch-like protein 38",
  "term_id": "GO:0005737",
  "term_label": "cytoplasm",
  "gene": "UniProtKB:Q2WGJ6"
}